{
  "gene": "UniProtKB:Q9UEU0",
  "gene_symbol": "VTI1B",
  "term_id": "GO:0006891",
  "gene_name": "Vesicle transport through interaction with t-SNAREs homolog 1B",
  "term_label": "intra-Golgi vesicle-mediated transport"
}